{
  "gene_name": "Proteasome subunit beta type-4",
  "term_id": "GO:0019774",
  "term_label": "proteasome core complex, beta-subunit complex",
  "gene_symbol": "PSMB4",
  "gene": "UniProtKB:P28070"
}